{
  "gene_name": "Stress-associated endoplasmic reticulum protein 2",
  "gene_symbol": "SERP2",
  "term_label": "Unknown molecular function",
  "gene": "UniProtKB:Q8N6R1",
  "term_id": "UNKNOWN:0001"
}